ceramide catabolic process [GO:0046514] (biological process) Sources: GOC:ai Definition: The chemical reactions and pathways resulting in the breakdown of ceramides, any N-acetylated sphingoid. Subtypes: ganglioside catabolic process [GO:0006689], GO:0046477 Relationships: is a type of ceramide metabolic process [GO:0006672]; is a type of sphingolipid catabolic process [GO:0030149] Also known as: ceramide breakdown, ceramide catabolism, ceramide degradation